{
  "term_label": "Unknown molecular function",
  "term_id": "UNKNOWN:0001",
  "gene": "UniProtKB:Q96MG7",
  "gene_name": "Non-structural maintenance of chromosomes element 3 homolog",
  "gene_symbol": "NSMCE3"
}